hydroxytrimethyllysine aldolase activity [GO:0120567] (molecular function) Relationships: is a type of GO:0016832 Definition: Catalysis of the reaction: (3S)-3-hydroxy-N(6),N(6),N(6)-trimethyl-L-lysine = 4-(trimethylamino)butanal + glycine. Also known as: HTMLA References: PMID:38615009 Sources: RHEA:79695